{
  "gene_name": "Tissue alpha-L-fucosidase",
  "gene": "UniProtKB:P04066",
  "gene_symbol": "FUCA1",
  "term_id": "GO:0005764",
  "term_label": "lysosome"
}